{
  "term_label": "ABC-type xenobiotic transporter activity",
  "gene": "UniProtKB:P33527",
  "term_id": "GO:0008559",
  "gene_name": "Multidrug resistance-associated protein 1",
  "gene_symbol": "ABCC1"
}